{
  "gene_name": "Keratin-associated protein 1-3",
  "gene": "UniProtKB:Q8IUG1",
  "gene_symbol": "KRTAP1-3",
  "term_label": "Unknown biological process",
  "term_id": "UNKNOWN:0002"
}